intracellular copper ion homeostasis [GO:0006878] (biological process) Also known as: copper homeostasis, cellular copper ion homeostasis Sources: GOC:ai, GOC:mah Definition: A homeostatic process involved in the maintenance of a steady state level of copper ions within a cell. Relationships: is a type of GO:0030003; is a type of copper ion homeostasis [GO:0055070]